{
  "gene_symbol": "LINC01548",
  "term_id": "UNKNOWN:0001",
  "term_label": "Unknown molecular function",
  "gene": "UniProtKB:A6NM66",
  "gene_name": "Uncharacterized protein encoded by LINC01548"
}